{
  "term_label": "postsynaptic density membrane",
  "term_id": "GO:0098839",
  "gene": "UniProtKB:Q9UF02",
  "gene_symbol": "CACNG5",
  "gene_name": "Voltage-dependent calcium channel gamma-5 subunit"
}